{
  "gene_name": "NADH-cytochrome b5 reductase 3",
  "term_label": "mitochondrion",
  "gene": "UniProtKB:P00387",
  "term_id": "GO:0005739",
  "gene_symbol": "CYB5R3"
}